centrosome separation [GO:0051299] (biological process) Subtypes: GO:0007100 Relationships: is a type of cell cycle process [GO:0022402]; is part of centrosome cycle [GO:0007098] Definition: The process in which duplicated centrosome components move away from each other. The centriole pair within each centrosome becomes part of a separate microtubule organizing center that nucleates a radial array of microtubules called an aster. The two asters move to opposite sides of the nucleus to form the two poles of the mitotic spindle. Sources: GOC:ai